{
  "gene_symbol": "GRB2",
  "gene": "UniProtKB:P62993",
  "term_label": "cytoplasm",
  "term_id": "GO:0005737",
  "gene_name": "Growth factor receptor-bound protein 2"
}